{
  "gene": "UniProtKB:Q9H1I8",
  "term_id": "GO:0006355",
  "term_label": "regulation of DNA-templated transcription",
  "gene_name": "Activating signal cointegrator 1 complex subunit 2",
  "gene_symbol": "ASCC2"
}